{
  "gene_name": "WD repeat-containing protein 47",
  "gene_symbol": "WDR47",
  "gene": "UniProtKB:O94967",
  "term_id": "UNKNOWN:0001",
  "term_label": "Unknown molecular function"
}